{
  "gene_symbol": "ATMIN",
  "term_id": "GO:0005634",
  "gene": "UniProtKB:O43313",
  "term_label": "nucleus",
  "gene_name": "ATM interactor"
}